{
  "gene_symbol": "C19orf25",
  "gene_name": "UPF0449 protein C19orf25",
  "term_id": "UNKNOWN:0002",
  "term_label": "Unknown biological process",
  "gene": "UniProtKB:Q9UFG5"
}